multi-species biofilm formation [GO:0044399] (biological process) Definition: A process in which planktonically growing microorganisms of different species grow at a liquid-air interface or on a solid substrate under the flow of a liquid and produce extracellular polymers that facilitate matrix formation, resulting in a change in the organisms' growth rate and gene transcription. Sources: GOC:cc, GOC:di, GOC:tb Also known as: multi-species biofilm formation in or on host organism, multi-species biofilm formation on inanimate substrate, multi-species submerged biofilm formation, multi-species surface biofilm formation Relationships: is a type of biofilm formation [GO:0042710]; is a type of biological process involved in symbiotic interaction [GO:0044403]